{
  "term_label": "mitotic cell cycle",
  "gene_symbol": "TUBA8",
  "gene_name": "Tubulin alpha-8 chain",
  "term_id": "GO:0000278",
  "gene": "UniProtKB:Q9NY65"
}